regulation of reticulophagy [GO:0140500] (biological process) Definition: Any process that modulates the frequency, rate or extent of reticulophagy. Relationships: is a type of regulation of macroautophagy [GO:0016241]; regulates reticulophagy [GO:0061709] Also known as: regulation of ER autophagy, regulation of ER-phagy, regulation of autophagy of the ER, regulation of autophagy of the endoplasmic reticulum, regulation of endoplasmic reticulum autophagy, regulation of ER degradation, regulation of endoplasmic reticulum degradation References: PMID:32735772 Subtypes: positive regulation of reticulophagy [GO:0140501]